{
  "term_id": "UNKNOWN:0003",
  "gene": "UniProtKB:Q14093",
  "term_label": "Unknown cellular component",
  "gene_name": "Cylicin-2",
  "gene_symbol": "CYLC2"
}